{
  "term_id": "GO:0000981",
  "term_label": "DNA-binding transcription factor activity, RNA polymerase II-specific",
  "gene_symbol": "ETV4",
  "gene": "UniProtKB:P43268",
  "gene_name": "ETS translocation variant 4"
}